taste receptor binding [GO:0031883] (molecular function) Sources: GOC:mah, GOC:nln Relationships: is a type of G protein-coupled receptor binding [GO:0001664] Subtypes: GO:0031884, type 1 member 2 taste receptor binding [GO:0031885], GO:0031886 Definition: Binding to a taste receptor. Also known as: taste receptor ligand